{
  "gene": "UniProtKB:P43119",
  "gene_symbol": "PTGIR",
  "term_id": "GO:0048662",
  "gene_name": "Prostacyclin receptor",
  "term_label": "negative regulation of smooth muscle cell proliferation"
}